{
  "gene_symbol": "USP51",
  "term_label": "Unknown molecular function",
  "gene_name": "Ubiquitin carboxyl-terminal hydrolase 51",
  "gene": "UniProtKB:Q70EK9",
  "term_id": "UNKNOWN:0001"
}